metanephric nephron tubule epithelial cell differentiation [GO:0072257] (biological process) Sources: GOC:mtg_kidney_jan10 Definition: The process in which relatively unspecialized cells acquire specialized structural and/or functional features that characterize the cells of the metanephric nephron tubule as it progresses from its formation to the mature state. Regulation: regulated by GO:0072307; negatively regulated by negative regulation of metanephric nephron tubule epithelial cell differentiation [GO:0072308] Relationships: is a type of GO:0072160; is a type of cell differentiation involved in metanephros development [GO:0072202]; is part of metanephric nephron tubule development [GO:0072234]